{
  "gene_symbol": "ACP5",
  "term_id": "GO:0003993",
  "term_label": "acid phosphatase activity",
  "gene": "UniProtKB:P13686",
  "gene_name": "Tartrate-resistant acid phosphatase type 5"
}